DDT-dehydrochlorinase activity [GO:0018833] (molecular function) Definition: Catalysis of the reaction: 1,1,1-trichloro-2,2-bis(4-chlorophenyl)ethane = 1,1-dichloro-2,2-bis(4-chlorophenyl)ethylene + chloride + H+. Sources: EC:4.5.1.1, RHEA:19217 Also known as: DDT dehydrochlorinase activity, 1,1,1-trichloro-2,2-bis(4-chlorophenyl)ethane chloride-lyase [1,1-dichloro-2,2-bis(4-chlorophenyl)ethylene-forming], 1,1,1-trichloro-2,2-bis(4-chlorophenyl)ethane chloride-lyase activity, DDT-as, DDT-ase activity, DDTase activity Relationships: is_a carbon-halide lyase activity [GO:0016848]